{
  "gene_name": "Calmodulin-like protein 5",
  "term_label": "calcium ion binding",
  "gene_symbol": "CALML5",
  "term_id": "GO:0005509",
  "gene": "UniProtKB:Q9NZT1"
}